{
  "term_label": "L-serine-pyruvate transaminase activity",
  "gene": "UniProtKB:P21549",
  "term_id": "GO:0004760",
  "gene_name": "Alanine--glyoxylate aminotransferase",
  "gene_symbol": "AGXT"
}